{
  "term_label": "nucleus",
  "gene_name": "G2_mitotic-specific cyclin-B1",
  "gene": "UniProtKB:P14635",
  "term_id": "GO:0005634",
  "gene_symbol": "CCNB1"
}